{
  "term_id": "GO:0051015",
  "gene_name": "Xin actin-binding repeat-containing protein 2",
  "gene_symbol": "XIRP2",
  "term_label": "actin filament binding",
  "gene": "UniProtKB:A4UGR9"
}